{
  "gene_symbol": "CD1D",
  "gene_name": "Antigen-presenting glycoprotein CD1d",
  "term_id": "GO:0009897",
  "gene": "UniProtKB:P15813",
  "term_label": "external side of plasma membrane"
}